{
  "gene": "UniProtKB:Q9NR33",
  "gene_symbol": "POLE4",
  "term_label": "DNA-templated DNA replication",
  "term_id": "GO:0006261",
  "gene_name": "DNA polymerase epsilon subunit 4"
}